{
  "gene_symbol": "ARL10",
  "term_label": "Unknown molecular function",
  "term_id": "UNKNOWN:0001",
  "gene_name": "ADP-ribosylation factor-like protein 10",
  "gene": "UniProtKB:Q8N8L6"
}